multidimensional cell growth [GO:0009825] (biological process) Definition: The process in which a cell irreversibly increases in size in two or three [spatial] dimensions or along two or three axes. Relationships: is a type of cell growth [GO:0016049] Sources: ISBN:0943088399 Also known as: cell growth in three dimensions, cell growth in two dimensions